{
  "term_id": "GO:0003735",
  "gene_symbol": "RPS8",
  "gene_name": "Small ribosomal subunit protein eS8",
  "gene": "UniProtKB:P62241",
  "term_label": "structural constituent of ribosome"
}